female germ-line sex determination [GO:0019099] (biological process) Definition: The determination of sex and sexual phenotype in a female organism's germ line. Sources: GOC:mah Also known as: sex determination, female germ-line determination Relationships: is a type of primary sex determination, germ-line [GO:0007542]; is a type of germ-line sex determination [GO:0018992]; is a type of female sex determination [GO:0030237]